{
  "term_id": "GO:0007186",
  "gene_name": "Cholecystokinin receptor type A",
  "gene_symbol": "CCKAR",
  "term_label": "G protein-coupled receptor signaling pathway",
  "gene": "UniProtKB:P32238"
}